{
  "gene_name": "Clusterin-like protein 1",
  "gene_symbol": "CLUL1",
  "gene": "UniProtKB:Q15846",
  "term_id": "GO:0005615",
  "term_label": "extracellular space"
}